{
  "term_id": "GO:0005634",
  "gene": "UniProtKB:O00401",
  "term_label": "nucleus",
  "gene_name": "Actin nucleation-promoting factor WASL",
  "gene_symbol": "WASL"
}